DNA cytosine deamination [GO:0070383] (biological process) Relationships: is a type of DNA deamination [GO:0045006] Definition: The removal of an amino group from a cytosine residue in DNA, forming a uracil residue. Sources: GOC:mah